{
  "gene_symbol": "REEP4",
  "term_id": "GO:0071786",
  "gene_name": "Receptor expression-enhancing protein 4",
  "gene": "UniProtKB:Q9H6H4",
  "term_label": "endoplasmic reticulum tubular network organization"
}